{
  "gene_name": "Tetratricopeptide repeat protein 33",
  "gene": "UniProtKB:Q6PID6",
  "term_id": "UNKNOWN:0001",
  "term_label": "Unknown molecular function",
  "gene_symbol": "TTC33"
}